{
  "term_label": "phosphatidylinositol 3-kinase/protein kinase B signal transduction",
  "gene_symbol": "C1orf54",
  "gene": "UniProtKB:Q8WWF1",
  "term_id": "GO:0043491",
  "gene_name": "Uncharacterized protein C1orf54"
}